nuclear migration along microtubule [GO:0030473] (biological process) Definition: The directed movement of the nucleus along microtubules within the cell, mediated by motor proteins. Subtypes: nuclear migration involved in conjugation with cellular fusion [GO:0000743], nucleokinesis involved in cell motility in cerebral cortex radial glia guided migration [GO:0021817], dynein-driven meiotic oscillatory nuclear movement [GO:0030989], nuclear migration during mitotic telophase [GO:0090561] Regulation: regulated by regulation of nuclear migration along microtubule [GO:1902838]; negatively regulated by negative regulation of nuclear migration along microtubule [GO:1902839]; positively regulated by GO:1902840 Also known as: nuclear movement, microtubule-mediated, nucleus migration, microtubule cytoskeleton-dependent nuclear positioning, microtubule cytoskeleton-dependent nucleus positioning, microtubule-dependent nuclear positioning, microtubule-dependent nucleus positioning, microtubule-mediated nuclear migration, nuclear migration, microtubule-mediated, transport of nucleus by microtubules, transport of nucleus, microtubule-mediated Sources: GOC:mah, GOC:sgd_curators Relationships: is a type of nuclear migration [GO:0007097]; is a type of GO:0072384